{
  "gene_symbol": "TAAR9",
  "term_label": "G protein-coupled receptor signaling pathway",
  "term_id": "GO:0007186",
  "gene_name": "Trace amine-associated receptor 9",
  "gene": "UniProtKB:Q96RI9"
}